[cytochrome c]-lysine N-methyltransferase activity [GO:0000277] (MF) Sources: EC:2.1.1.59 Also known as: S-adenosyl-L-methionine:cytochrome c-L-lysine 6-N-methyltransferase activity, S-adenosyl-L-methionine:cytochrome c-L-lysine N6-methyltransferase activity, cytochrome c (lysine) methyltransferase activity, cytochrome c methyltransferase activity, cytochrome c-lysine N-methyltransferase activity, cytochrome c-specific protein methylase III activity, cytochrome c-specific protein-lysine methyltransferase activity Relationships: is a type of protein-lysine N-methyltransferase activity [GO:0016279] Definition: Catalysis of the reaction: S-adenosyl-L-methionine + cytochrome c L-lysine = S-adenosyl-L-homocysteine + cytochrome c N6-methyl-L-lysine. This is the addition of a methyl group to the N6 atom of a lysine residue in cytochrome c.